{
  "gene_name": "Active regulator of SIRT1",
  "term_label": "enzyme binding",
  "term_id": "GO:0019899",
  "gene_symbol": "RPS19BP1",
  "gene": "UniProtKB:Q86WX3"
}